{
  "gene_symbol": "QARS1",
  "term_label": "glutamine-tRNA ligase activity",
  "gene_name": "Glutamine--tRNA ligase",
  "term_id": "GO:0004819",
  "gene": "UniProtKB:P47897"
}